{
  "gene": "UniProtKB:Q49A88",
  "gene_name": "Coiled-coil domain-containing protein 14",
  "gene_symbol": "CCDC14",
  "term_label": "centriolar satellite",
  "term_id": "GO:0034451"
}